{
  "term_label": "nucleus",
  "gene_name": "EZH inhibitory protein",
  "term_id": "GO:0005634",
  "gene_symbol": "EZHIP",
  "gene": "UniProtKB:Q86X51"
}